maternal mRNA clearance [GO:0141065] (biological process) Also known as: maternal mRNA degradation, maternal transcript clearance, maternal transcript degradation References: PMID:19204068, PMID:32558204 Relationships: is a type of GO:0006402; is part of maternal-to-zygotic transition of gene expression [GO:0160021] Definition: The chemical reactions and pathways resulting in the clearance of maternal mRNA transcripts from the zygote as part of the maternal-to-zygote transition in gene expression.